{
  "gene_symbol": "ANP32E",
  "term_label": "regulation of apoptotic process",
  "gene_name": "Acidic leucine-rich nuclear phosphoprotein 32 family member E",
  "term_id": "GO:0042981",
  "gene": "UniProtKB:Q9BTT0"
}